{
  "term_id": "GO:0006338",
  "gene_name": "Chromodomain-helicase-DNA-binding protein 7",
  "term_label": "chromatin remodeling",
  "gene_symbol": "CHD7",
  "gene": "UniProtKB:Q9P2D1"
}